{
  "gene": "UniProtKB:Q969F9",
  "gene_symbol": "HPS3",
  "term_id": "GO:0005737",
  "term_label": "cytoplasm",
  "gene_name": "BLOC-2 complex member HPS3"
}